{
  "gene_name": "2-oxoisovalerate dehydrogenase subunit alpha, mitochondrial",
  "term_id": "GO:0160157",
  "gene": "UniProtKB:P12694",
  "gene_symbol": "BCKDHA",
  "term_label": "branched-chain alpha-ketoacid dehydrogenase complex"
}